{
  "gene_symbol": "RSRC1",
  "gene": "UniProtKB:Q96IZ7",
  "gene_name": "Serine_Arginine-related protein 53",
  "term_label": "Unknown molecular function",
  "term_id": "UNKNOWN:0001"
}